ATP-binding cassette (ABC) transporter complex, substrate-binding subunit-containing [GO:0055052] (cellular component) Sources: GOC:mlg, GOC:mtg_sensu Definition: A complex for the transport of metabolites into the cell, consisting of 5 subunits: two ATP-binding subunits, two membrane spanning subunits, and one substrate-binding subunit. In organisms with two membranes, the substrate-binding protein moves freely in the periplasmic space and joins the other subunits only when bound with substrate. In organisms with only one membrane the substrate-binding protein is tethered to the cytoplasmic membrane and associated with the other subunits. Transport of the substrate across the membrane is driven by the hydrolysis of ATP. Relationships: is a type of ATP-binding cassette (ABC) transporter complex [GO:0043190]